{
  "gene_symbol": "AKR1C4",
  "gene": "UniProtKB:P17516",
  "term_id": "GO:0032052",
  "term_label": "bile acid binding",
  "gene_name": "Aldo-keto reductase family 1 member C4"
}